{
  "term_id": "GO:0016192",
  "term_label": "vesicle-mediated transport",
  "gene_name": "AP-2 complex subunit sigma",
  "gene": "UniProtKB:P53680",
  "gene_symbol": "AP2S1"
}